{
  "gene_name": "Solute carrier family 35 member D3",
  "term_label": "antiporter activity",
  "term_id": "GO:0015297",
  "gene": "UniProtKB:Q5M8T2",
  "gene_symbol": "SLC35D3"
}